{
  "gene_symbol": "TLX1NB",
  "gene_name": "Putative TLX1 neighbor protein",
  "term_label": "Unknown molecular function",
  "term_id": "UNKNOWN:0001",
  "gene": "UniProtKB:P0CAT3"
}